{
  "gene_name": "TIR domain-containing adapter molecule 2",
  "term_id": "GO:0043123",
  "term_label": "positive regulation of canonical NF-kappaB signal transduction",
  "gene_symbol": "TICAM2",
  "gene": "UniProtKB:Q86XR7"
}